{
  "gene": "UniProtKB:Q8NI36",
  "gene_symbol": "WDR36",
  "term_id": "GO:0034388",
  "gene_name": "WD repeat-containing protein 36",
  "term_label": "Pwp2p-containing subcomplex of 90S preribosome"
}